{
  "gene_name": "Cytochrome P450 2U1",
  "gene": "UniProtKB:Q7Z449",
  "term_id": "GO:0016712",
  "gene_symbol": "CYP2U1",
  "term_label": "oxidoreductase activity, acting on paired donors, with incorporation or reduction of molecular oxygen, reduced flavin or flavoprotein as one donor, and incorporation of one atom of oxygen"
}